{
  "term_id": "UNKNOWN:0003",
  "gene": "UniProtKB:Q96I15",
  "gene_symbol": "SCLY",
  "gene_name": "Selenocysteine lyase",
  "term_label": "Unknown cellular component"
}